RNA polymerase II CTD heptapeptide repeat P3 isomerase activity [GO:0140839] (MF) References: PMID:28248323 Definition: Catalysis of the reaction: RNA polymerase II large subunit CTD heptapeptide repeat (consensus YSPTSPS) cis-proline (omega=180) (position 3) = RNA polymerase II large subunit trans-proline (omega=0) (position 3). Relationships: is a type of RNA polymerase II CTD heptapeptide repeat peptidyl-prolyl isomerase activity [GO:0140838] Also known as: RNA polymerase II C-terminal domain P3 isomerase activity